{
  "gene": "UniProtKB:Q96LP6",
  "term_label": "Unknown cellular component",
  "gene_symbol": "C12orf42",
  "term_id": "UNKNOWN:0003",
  "gene_name": "Uncharacterized protein C12orf42"
}